taxoid 14-beta-hydroxylase activity [GO:0036203] (molecular function) Definition: Catalysis of the reaction: 10beta-hydroxytaxa-4(20),11-dien-5alpha-yl acetate + O2 + NADPH + H+ = 10beta,14beta-dihydroxytaxa-4(20),11-dien-5alpha-yl acetate + NADP+ + H2O. Relationships: is a type of GO:0016709 Sources: EC:1.14.13.146